{
  "gene": "UniProtKB:P58557",
  "term_label": "RNA endonuclease activity",
  "gene_name": "Endoribonuclease YbeY",
  "term_id": "GO:0004521",
  "gene_symbol": "YBEY"
}